{
  "gene_name": "Ventral anterior homeobox 2",
  "term_label": "RNA polymerase II cis-regulatory region sequence-specific DNA binding",
  "gene_symbol": "VAX2",
  "gene": "UniProtKB:Q9UIW0",
  "term_id": "GO:0000978"
}